inward rectifying potassium channel [GO:0008282] (cellular component) Definition: A protein complex that comprises four pore-forming (Kir6.x) and four regulatory sulphonylurea receptor (SURx) subunits and forms a transmembrane channel through which ions may pass. The opening and closing of the channel is regulated by ATP: binding of ATP to the Kir6.x subunit inhibits channel activity, whereas binding of Mg2+-complexed ATP or ADP to the SURx subunit stimulates channel activity. Relationships: is a type of potassium channel complex [GO:0034705]; is a type of plasma membrane protein complex [GO:0098797] References: PMID:16308567, PMID:16956886 Sources: GOC:bhm Also known as: ATP-sensitive potassium channel complex, inward rectifying K+ channel, KCNJ11-SUR complex, KCNJ11-SURx complex, KCNJ8-SUR complex, KCNJ8-SURx complex, Kir6-SUR complex, Kir6.1-SUR complex, Kir6.1-SURx complex, Kir6.2-SUR complex, Kir6.2-SURx complex, Kir6.x complex, Kir6.x-SURx complex